regulation of glucocorticoid catabolic process [GO:0031949] (BP) Sources: GOC:mah Definition: Any process that modulates the frequency, rate or extent of the chemical reactions and pathways resulting in the breakdown of glucocorticoids. Relationships: is a type of regulation of glucocorticoid metabolic process [GO:0031943]; is a type of regulation of lipid catabolic process [GO:0050994]; regulates GO:0006713 Subtypes: negative regulation of glucocorticoid catabolic process [GO:0031950], GO:0031951